{
  "term_label": "fibroblast growth factor receptor binding",
  "gene": "UniProtKB:P05230",
  "gene_name": "Fibroblast growth factor 1",
  "gene_symbol": "FGF1",
  "term_id": "GO:0005104"
}